{
  "term_id": "GO:0003333",
  "gene": "UniProtKB:Q9HBR0",
  "gene_name": "Putative sodium-coupled neutral amino acid transporter 10",
  "term_label": "amino acid transmembrane transport",
  "gene_symbol": "SLC38A10"
}